{
  "term_id": "GO:0005789",
  "gene_name": "Junctophilin-3",
  "gene_symbol": "JPH3",
  "gene": "UniProtKB:Q8WXH2",
  "term_label": "endoplasmic reticulum membrane"
}